{
  "term_label": "histone deacetylase binding",
  "gene": "UniProtKB:Q9HCU9",
  "gene_symbol": "BRMS1",
  "term_id": "GO:0042826",
  "gene_name": "Breast cancer metastasis-suppressor 1"
}